positive regulation of oospore formation [GO:0075245] (biological process) Definition: Any process that activates, maintains or increases the frequency, rate or extent of oospore formation, a process in which male and female gametangia develop and fuse to form a thick-walled resting spore of oomycetes. Relationships: is a type of GO:0043941; is a type of regulation of oospore formation [GO:0075244]; positively regulates oospore formation [GO:0075243] Sources: GOC:pamgo_curators